{
  "gene_symbol": "MAFG",
  "gene_name": "Transcription factor MafG",
  "term_id": "GO:0006357",
  "gene": "UniProtKB:O15525",
  "term_label": "regulation of transcription by RNA polymerase II"
}